{
  "gene": "UniProtKB:P29084",
  "term_id": "GO:0001097",
  "gene_symbol": "GTF2E2",
  "term_label": "TFIIH-class transcription factor complex binding",
  "gene_name": "Transcription initiation factor IIE subunit beta"
}